{
  "gene_symbol": "ORC4",
  "term_label": "nuclear origin of replication recognition complex",
  "term_id": "GO:0005664",
  "gene_name": "Origin recognition complex subunit 4",
  "gene": "UniProtKB:O43929"
}